{
  "gene_symbol": "FUCA2",
  "gene": "UniProtKB:Q9BTY2",
  "term_id": "GO:0004560",
  "term_label": "alpha-L-fucosidase activity",
  "gene_name": "Plasma alpha-L-fucosidase"
}